regulation of timing of animal organ formation [GO:0048504] (biological process) Definition: Any process that modulates the rate, frequency or extent of animal organ formation at a consistent predetermined time point during development. Sources: GOC:bf, GOC:dph, GOC:jid, GOC:tb Relationships: is a type of regulation of animal organ formation [GO:0003156]; is a type of regulation of development, heterochronic [GO:0040034] Also known as: timing of organ biosynthesis, timing of organ formation